protein-arginine N-acetylglucosaminyltransferase activity [GO:0106362] (molecular function) Definition: Catalysis of the reaction: L-arginyl-[protein] + UDP-N-acetyl-alpha-D-glucosamine = H+ + N(omega)-(N-acetyl-beta-D-glucosaminyl)-L-arginyl-[protein] + UDP. Relationships: is a type of GO:0016262 References: PMID:23955153, PMID:30619781 Sources: GOC:sp, RHEA:66632